{
  "term_id": "GO:0005737",
  "term_label": "cytoplasm",
  "gene_name": "Dual specificity protein phosphatase 19",
  "gene_symbol": "DUSP19",
  "gene": "UniProtKB:Q8WTR2"
}